{
  "gene_name": "Calcium_calmodulin-dependent protein kinase type 1",
  "term_id": "GO:0005737",
  "gene_symbol": "CAMK1",
  "gene": "UniProtKB:Q14012",
  "term_label": "cytoplasm"
}